{
  "term_label": "G protein-coupled receptor signaling pathway",
  "gene": "UniProtKB:P63215",
  "term_id": "GO:0007186",
  "gene_name": "Guanine nucleotide-binding protein G(I)_G(S)_G(O) subunit gamma-3",
  "gene_symbol": "GNG3"
}